{
  "term_id": "UNKNOWN:0002",
  "gene_symbol": "ACP1",
  "term_label": "Unknown biological process",
  "gene_name": "Low molecular weight phosphotyrosine protein phosphatase",
  "gene": "UniProtKB:P24666"
}